{
  "gene_symbol": "ANKRD36",
  "term_label": "Unknown cellular component",
  "term_id": "UNKNOWN:0003",
  "gene": "UniProtKB:A6QL64",
  "gene_name": "Ankyrin repeat domain-containing protein 36A"
}